{
  "term_label": "DNA-binding transcription factor activity, RNA polymerase II-specific",
  "gene_symbol": "ZNF568",
  "gene": "UniProtKB:Q3ZCX4",
  "gene_name": "Zinc finger protein 568",
  "term_id": "GO:0000981"
}